{
  "gene_name": "Intraflagellar transport protein 88 homolog",
  "gene": "UniProtKB:Q13099",
  "term_id": "GO:0036064",
  "term_label": "ciliary basal body",
  "gene_symbol": "IFT88"
}